{
  "gene_symbol": "SOHLH1",
  "term_id": "GO:0000976",
  "gene": "UniProtKB:Q5JUK2",
  "term_label": "transcription cis-regulatory region binding",
  "gene_name": "Spermatogenesis- and oogenesis-specific basic helix-loop-helix-containing protein 1"
}